{
  "gene_name": "Aquaporin-7",
  "term_label": "plasma membrane",
  "term_id": "GO:0005886",
  "gene": "UniProtKB:O14520",
  "gene_symbol": "AQP7"
}